{
  "term_id": "GO:0005096",
  "gene": "UniProtKB:Q9BYX2",
  "gene_symbol": "TBC1D2",
  "term_label": "GTPase activator activity",
  "gene_name": "TBC1 domain family member 2A"
}